canonical Wnt signaling pathway involved in heart development [GO:0061316] (biological process) Definition: The series of molecular signals initiated by binding of a Wnt protein to a frizzled family receptor on the surface of the target cell, followed by propagation of the signal via beta-catenin, and ending with a change in transcription of target genes that contributes to the progression of the heart over time. In this pathway, the activated receptor signals via downstream effectors that result in the inhibition of beta-catenin phosphorylation, thereby preventing degradation of beta-catenin. Stabilized beta-catenin can then accumulate and travel to the nucleus to trigger changes in transcription of target genes. Sources: GOC:mtg_heart Also known as: canonical Wnt receptor signaling pathway involved in heart development, canonical Wnt receptor signalling pathway involved in heart development, canonical Wnt-activated signaling pathway involved in heart development Relationships: is a type of Wnt signaling pathway involved in heart development [GO:0003306]; is_a canonical Wnt signaling pathway [GO:0060070]